{
  "gene_symbol": "ZNF487",
  "gene": "UniProtKB:B1APH4",
  "term_label": "regulation of transcription by RNA polymerase II",
  "gene_name": "Putative zinc finger protein 487",
  "term_id": "GO:0006357"
}